{
  "gene": "UniProtKB:A2A368",
  "term_label": "negative regulation of transcription by RNA polymerase II",
  "gene_symbol": "MAGEB16",
  "term_id": "GO:0000122",
  "gene_name": "Melanoma-associated antigen B16"
}